{
  "gene": "UniProtKB:O43542",
  "gene_name": "DNA repair protein XRCC3",
  "term_id": "GO:0045003",
  "term_label": "double-strand break repair via synthesis-dependent strand annealing",
  "gene_symbol": "XRCC3"
}